regulation of neuromuscular synaptic transmission [GO:1900073] (BP) Subtypes: negative regulation of neuromuscular synaptic transmission [GO:1900074], GO:1900075 Sources: GOC:TermGenie, GOC:kmv Definition: Any process that modulates the frequency, rate or extent of neuromuscular synaptic transmission. Relationships: is a type of modulation of chemical synaptic transmission [GO:0050804]; regulates neuromuscular synaptic transmission [GO:0007274]